bis(5'-nucleosyl)-tetraphosphatase activity [GO:0008796] (molecular function) Subtypes: GO:0004081, bis(5'-nucleosyl)-tetraphosphatase (symmetrical) activity [GO:0008803] Relationships: is a type of pyrophosphatase activity [GO:0016462] Definition: Catalysis of the hydrolysis of P(1),P(4)-bis(5'-nucleosyl)tetraphosphate into two nucleotides. Sources: GOC:ai